{
  "gene_symbol": "FCGBP",
  "term_label": "extracellular matrix",
  "gene": "UniProtKB:Q9Y6R7",
  "gene_name": "IgGFc-binding protein",
  "term_id": "GO:0031012"
}